{
  "gene": "UniProtKB:Q6PGP7",
  "term_id": "GO:0055087",
  "gene_name": "Superkiller complex protein 3",
  "term_label": "Ski complex",
  "gene_symbol": "SKIC3"
}